phenylalanine 4-monooxygenase activity [GO:0004505] (molecular function) Definition: Catalysis of the reaction: L-phenylalanine + tetrahydrobiopterin + O2 = L-tyrosine + 4-alpha-hydroxytetrahydrobiopterin. Also known as: phenylalanine hydroxylase activity, L-phenylalanine,tetrahydrobiopterin:oxygen oxidoreductase (4-hydroxylating), PAH activity, phenylalaninase activity, phenylalanine 4-hydroxylase activity References: PMID:4004813 Sources: RHEA:20273 Relationships: is_a GO:0016714; is part of GO:0019293